{
  "gene_name": "Cyclin-dependent kinase 4",
  "gene": "UniProtKB:P11802",
  "term_id": "GO:0005634",
  "term_label": "nucleus",
  "gene_symbol": "CDK4"
}